{
  "gene_name": "Zinc finger protein 641",
  "term_id": "GO:0000977",
  "term_label": "RNA polymerase II transcription regulatory region sequence-specific DNA binding",
  "gene": "UniProtKB:Q96N77",
  "gene_symbol": "ZNF641"
}